{
  "gene": "UniProtKB:Q9HBH7",
  "gene_symbol": "BEX1",
  "gene_name": "Protein BEX1",
  "term_label": "cytoplasm",
  "term_id": "GO:0005737"
}